{
  "term_id": "GO:0006103",
  "gene_name": "Dihydrolipoyl dehydrogenase, mitochondrial",
  "term_label": "2-oxoglutarate metabolic process",
  "gene_symbol": "DLD",
  "gene": "UniProtKB:P09622"
}